{
  "term_id": "GO:0007166",
  "gene_name": "T cell receptor beta variable 9",
  "term_label": "cell surface receptor signaling pathway",
  "gene": "UniProtKB:A0A0B4J1U6",
  "gene_symbol": "TRBV9"
}